negative regulation of stem cell differentiation [GO:2000737] (biological process) Definition: Any process that stops, prevents or reduces the frequency, rate or extent of stem cell differentiation. Subtypes: negative regulation of cardioblast differentiation [GO:0051892], negative regulation of hematopoietic stem cell differentiation [GO:1902037], negative regulation of neural crest cell differentiation [GO:1905293], negative regulation of mesenchymal stem cell differentiation [GO:2000740] Relationships: is_a negative regulation of cell differentiation [GO:0045596]; is a type of regulation of stem cell differentiation [GO:2000736]; RO_0002212 GO:0048863 Sources: GOC:obol